{
  "gene_name": "DNA dC-dU-editing enzyme APOBEC-3F",
  "gene": "UniProtKB:Q8IUX4",
  "term_label": "negative regulation of single stranded viral RNA replication via double stranded DNA intermediate",
  "gene_symbol": "APOBEC3F",
  "term_id": "GO:0045869"
}